{
  "term_id": "GO:0003713",
  "gene_name": "Core-binding factor subunit beta",
  "gene_symbol": "CBFB",
  "gene": "UniProtKB:Q13951",
  "term_label": "transcription coactivator activity"
}